meiotic cell cycle [GO:0051321] (biological process) Definition: Progression through the phases of the meiotic cell cycle, in which canonically a cell replicates to produce four offspring with half the chromosomal content of the progenitor cell via two nuclear divisions. Sources: GOC:ai Also known as: meiosis Note: Note that this term should not be confused with 'GO:0140013 ; meiotic nuclear division'. 'GO:0051321 ; meiotic cell cycle represents the entire mitotic cell cycle, while 'GO:0140013 meiotic nuclear division' specifically represents the actual nuclear division step of the mitotic cell cycle. Relationships: is a type of cell cycle [GO:0007049]; is a type of GO:0022414; is part of sexual reproduction [GO:0019953]; has part GO:0140013 Subtypes: GO:0048236 Regulation: regulated by regulation of meiotic cell cycle [GO:0051445]; positively regulated by positive regulation of meiotic cell cycle [GO:0051446]; negatively regulated by negative regulation of meiotic cell cycle [GO:0051447]